{
  "gene_name": "Phosphoglycerate kinase 2",
  "term_id": "GO:0006096",
  "gene_symbol": "PGK2",
  "term_label": "glycolytic process",
  "gene": "UniProtKB:P07205"
}